fibroblast growth factor receptor signaling pathway involved in forebrain neuroblast division [GO:0021875] (biological process) Relationships: is_a fibroblast growth factor receptor signaling pathway [GO:0008543]; is part of forebrain neuroblast division [GO:0021873] Definition: The series of molecular signals generated as a consequence of a fibroblast growth factor receptor binding to one of its physiological ligands that contributes to the self renewal of neuroblasts in the forebrain. Also known as: fibroblast growth factor receptor signalling pathway in forebrain neuroblast division References: PMID:16226447 Sources: GOC:cls, GOC:dgh, GOC:dph, GOC:jid, GO_REF:0000021